{
  "gene": "UniProtKB:Q9UJU5",
  "gene_name": "Forkhead box protein D3",
  "term_label": "anatomical structure morphogenesis",
  "term_id": "GO:0009653",
  "gene_symbol": "FOXD3"
}